{
  "gene_symbol": "HOOK1",
  "gene_name": "Protein Hook homolog 1",
  "gene": "UniProtKB:Q9UJC3",
  "term_id": "GO:0008017",
  "term_label": "microtubule binding"
}